protein-N(PI)-phosphohistidine-mannose phosphotransferase system transporter activity [GO:0022870] (molecular function) Also known as: mannose PTS transporter activity Relationships: is a type of protein-N(PI)-phosphohistidine-sugar phosphotransferase activity [GO:0008982]; is a type of mannose transmembrane transporter activity [GO:0015578] Definition: Catalysis of the PEP-dependent, phosphoryl transfer-driven transport of substances across a membrane. The transport happens by catalysis of the reaction: protein N-phosphohistidine + mannose(out) = protein histidine + mannose phosphate(in). This differs from primary and secondary active transport in that the solute is modified during transport. Sources: GOC:mtg_transport, ISBN:0815340729